{
  "gene": "UniProtKB:Q5VWZ2",
  "term_label": "palmitoyl-(protein) hydrolase activity",
  "gene_symbol": "LYPLAL1",
  "term_id": "GO:0008474",
  "gene_name": "Lysophospholipase-like protein 1"
}